interchromatin granule [GO:0035061] (cellular component) Definition: A class of nuclear body measuring 20-25 nm in diameter and distributed throughout the interchromatin space, linked together by thin fibrils. They are believed to be storage centers for various snRNAs, snRNPs, serine/arginine-rich proteins and RNA polymerase II. A typical mammalian cell contains 25-50 clusters of interchromatin granules. Interchromatin granule clusters do not contain the heterogeneous nuclear RNA-binding proteins (hnRNPs). Relationships: is a type of nuclear body [GO:0016604] Also known as: ICG References: PMID:10984439 Sources: GOC:bf